{
  "term_label": "ubiquitin protein ligase activity",
  "gene_symbol": "RNF34",
  "gene_name": "E3 ubiquitin-protein ligase RNF34",
  "gene": "UniProtKB:Q969K3",
  "term_id": "GO:0061630"
}